positive regulation of basophil differentiation [GO:0045642] (biological process) Also known as: up regulation of basophil differentiation, up-regulation of basophil differentiation, upregulation of basophil differentiation, activation of basophil differentiation, stimulation of basophil differentiation Sources: GOC:go_curators Definition: Any process that activates or increases the frequency, rate or extent of basophil differentiation. Relationships: is a type of positive regulation of granulocyte differentiation [GO:0030854]; is a type of regulation of basophil differentiation [GO:0045640]; positively regulates GO:0030221